{
  "gene": "UniProtKB:A0A1B0GUA7",
  "term_label": "Unknown biological process",
  "term_id": "UNKNOWN:0002",
  "gene_symbol": "TEX51",
  "gene_name": "Testis-expressed protein 51"
}